{
  "gene_symbol": "SERPINI1",
  "term_label": "Unknown biological process",
  "gene": "UniProtKB:Q99574",
  "gene_name": "Neuroserpin",
  "term_id": "UNKNOWN:0002"
}